adenine biosynthetic process [GO:0046084] (biological process) Subtypes: adenine salvage [GO:0006168] Sources: GOC:go_curators Also known as: adenine anabolism, adenine biosynthesis, adenine formation, adenine synthesis Regulation: regulated by regulation of adenine biosynthetic process [GO:0061934] Definition: The chemical reactions and pathways resulting in the formation of adenine, 6-aminopurine, one of the five main bases found in nucleic acids and a component of numerous important derivatives of its corresponding ribonucleoside, adenosine. Relationships: is a type of GO:0009113; is a type of adenine metabolic process [GO:0046083]